{
  "term_label": "signaling receptor binding",
  "gene_name": "V-set domain-containing T-cell activation inhibitor 1",
  "term_id": "GO:0005102",
  "gene": "UniProtKB:Q7Z7D3",
  "gene_symbol": "VTCN1"
}